{
  "gene_symbol": "ARK2C",
  "term_id": "GO:0005634",
  "gene": "UniProtKB:Q6ZSG1",
  "term_label": "nucleus",
  "gene_name": "E3 ubiquitin-protein ligase ARK2C"
}